{
  "term_id": "GO:0005634",
  "gene": "UniProtKB:A0A494C1R9",
  "gene_symbol": "TSPY9",
  "term_label": "nucleus",
  "gene_name": "Testis-specific Y-encoded protein 9"
}